{
  "term_label": "potassium ion transmembrane transport",
  "gene_name": "Potassium voltage-gated channel subfamily A member 6",
  "gene": "UniProtKB:P17658",
  "term_id": "GO:0071805",
  "gene_symbol": "KCNA6"
}